regulation of morphogenesis of a branching structure [GO:0060688] (biological process) Sources: GOC:dph Subtypes: regulation of prostatic bud formation [GO:0060685], regulation of branching involved in prostate gland morphogenesis [GO:0060687], regulation of branching involved in salivary gland morphogenesis [GO:0060693], regulation of branching involved in mammary gland duct morphogenesis [GO:0060762], GO:0061046, pancreas induction [GO:0061132], regulation of branching involved in ureteric bud morphogenesis [GO:0090189], GO:1905553, regulation of secondary shoot formation [GO:2000032], GO:2000172 Relationships: is a type of GO:0022603; is a type of GO:0051239; regulates morphogenesis of a branching structure [GO:0001763] Definition: Any process that modulates the rate, frequency, or extent of branching morphogenesis, the process in which the anatomical structures of branches are generated and organized.